{
  "gene_name": "CUB domain-containing protein 2",
  "gene_symbol": "CDCP2",
  "term_label": "Unknown cellular component",
  "term_id": "UNKNOWN:0003",
  "gene": "UniProtKB:Q5VXM1"
}